{
  "gene_name": "Epidermal growth factor receptor",
  "term_id": "GO:0043410",
  "gene_symbol": "EGFR",
  "gene": "UniProtKB:P00533",
  "term_label": "positive regulation of MAPK cascade"
}